{
  "term_id": "GO:0008074",
  "gene": "UniProtKB:Q02153",
  "gene_symbol": "GUCY1B1",
  "term_label": "guanylate cyclase complex, soluble",
  "gene_name": "Guanylate cyclase soluble subunit beta-1"
}